{
  "gene_symbol": "BORA",
  "gene": "UniProtKB:Q6PGQ7",
  "term_label": "protein kinase binding",
  "gene_name": "Protein aurora borealis",
  "term_id": "GO:0019901"
}